{
  "gene_symbol": "ARV1",
  "gene": "UniProtKB:Q9H2C2",
  "gene_name": "Protein ARV1",
  "term_label": "regulation of plasma membrane sterol distribution",
  "term_id": "GO:0097036"
}